{
  "term_label": "Unknown molecular function",
  "gene": "UniProtKB:Q8IXX5",
  "term_id": "UNKNOWN:0001",
  "gene_symbol": "TMEM183A",
  "gene_name": "Transmembrane protein 183A"
}